{
  "term_id": "GO:0005093",
  "gene_name": "Rab GDP dissociation inhibitor alpha",
  "term_label": "Rab GDP-dissociation inhibitor activity",
  "gene_symbol": "GDI1",
  "gene": "UniProtKB:P31150"
}